{
  "gene_symbol": "FHIT",
  "gene": "UniProtKB:P49789",
  "term_id": "GO:0032435",
  "term_label": "negative regulation of proteasomal ubiquitin-dependent protein catabolic process",
  "gene_name": "Bis(5'-adenosyl)-triphosphatase"
}